labd-13Z-ene-9,15,16-triol synthase activity [GO:0106240] (molecular function) References: PMID:29315936 Sources: GOC:eab, RHEA:62192 Definition: Catalysis of the reaction: O2 + peregrinol + reduced [NADPH--hemoprotein reductase] = H+ + H2O + labd-13Z-ene-9,15,16-triol + oxidized [NADPH--hemoprotein reductase]. Relationships: is a type of GO:0016712